{
  "gene_symbol": "SCAP",
  "term_label": "Unknown molecular function",
  "gene_name": "Sterol regulatory element-binding protein cleavage-activating protein",
  "term_id": "UNKNOWN:0001",
  "gene": "UniProtKB:Q12770"
}